2-oxoaldehyde dehydrogenase (NADP+) activity [GO:0047552] (molecular function) Relationships: is a type of aldehyde dehydrogenase (NADP+) activity [GO:0033721] Sources: RHEA:18129 Definition: Catalysis of the reaction: a 2-oxoaldehyde + NADP+ + H2O = a 2-oxo acid + NADPH + H+. Also known as: 2-ketoaldehyde dehydrogenase, alpha-ketoaldehyde dehydrogenase activity, methylglyoxal dehydrogenase activity, 2-oxoaldehyde:NADP+ 2-oxidoreductase activity, NADP-dependent alpha-ketoaldehyde dehydrogenase activity, NADP-linked alpha-ketoaldehyde dehydrogenase activity